{
  "term_label": "macroautophagy",
  "gene": "UniProtKB:Q9H6K1",
  "gene_symbol": "ILRUN",
  "term_id": "GO:0016236",
  "gene_name": "Protein ILRUN"
}